{
  "term_id": "GO:0001916",
  "gene": "UniProtKB:P04439",
  "gene_name": "HLA class I histocompatibility antigen, A alpha chain",
  "gene_symbol": "HLA-A",
  "term_label": "positive regulation of T cell mediated cytotoxicity"
}